{
  "gene_symbol": "CENPK",
  "term_id": "UNKNOWN:0003",
  "gene": "UniProtKB:Q9BS16",
  "gene_name": "Centromere protein K",
  "term_label": "Unknown cellular component"
}